kinesin I complex [GO:0016938] (cellular component) Definition: A complex of two kinesin heavy chains and two kinesin light chains. References: PMID:20930137 Relationships: is_a kinesin complex [GO:0005871]